hydroxymethyl-, formyl- and related transferase activity [GO:0016742] (molecular function) Subtypes: 3-methyl-2-oxobutanoate hydroxymethyltransferase activity [GO:0003864], GO:0004047, GO:0004372, methionyl-tRNA formyltransferase activity [GO:0004479], phosphoribosylaminoimidazolecarboxamide formyltransferase activity [GO:0004643], phosphoribosylglycinamide formyltransferase activity [GO:0004644], glycine formimidoyltransferase activity [GO:0030408], glutamate formimidoyltransferase activity [GO:0030409], deoxycytidylate 5-hydroxymethyltransferase activity [GO:0047153], D-alanine 2-hydroxymethyltransferase activity [GO:0050413], UDP-4-amino-4-deoxy-L-arabinose formyltransferase activity [GO:0099619] Relationships: is a type of transferase activity, transferring one-carbon groups [GO:0016741] Sources: EC:2.1.2.-, GOC:mah Definition: Catalysis of the transfer of a hydroxymethyl- or formyl group from one compound (donor) to another (acceptor).